{
  "gene_symbol": "UBE2A",
  "gene": "UniProtKB:P49459",
  "term_label": "ubiquitin conjugating enzyme activity",
  "term_id": "GO:0061631",
  "gene_name": "Ubiquitin-conjugating enzyme E2 A"
}